{
  "term_id": "GO:0005829",
  "gene_name": "Glycogen synthase kinase-3 alpha",
  "term_label": "cytosol",
  "gene": "UniProtKB:P49840",
  "gene_symbol": "GSK3A"
}